{
  "gene_symbol": "ISCU",
  "term_label": "intracellular iron ion homeostasis",
  "gene_name": "Iron-sulfur cluster assembly enzyme ISCU",
  "term_id": "GO:0006879",
  "gene": "UniProtKB:Q9H1K1"
}